{
  "term_label": "RNA polymerase II transcription regulatory region sequence-specific DNA binding",
  "gene_symbol": "ZNF674",
  "gene": "UniProtKB:Q2M3X9",
  "gene_name": "Zinc finger protein 674",
  "term_id": "GO:0000977"
}